{
  "term_id": "GO:0000139",
  "gene_name": "Proprotein convertase subtilisin_kexin type 4",
  "gene": "UniProtKB:Q6UW60",
  "gene_symbol": "PCSK4",
  "term_label": "Golgi membrane"
}